anaerobic phenol-containing compound catabolic process [GO:0046193] (biological process) Relationships: is_a phenol-containing compound catabolic process [GO:0019336]; is a type of anaerobic phenol-containing compound metabolic process [GO:0042215] Also known as: anaerobic phenol-containing compound breakdown, anaerobic phenol-containing compound catabolism, anaerobic phenol-containing compound degradation Definition: The chemical reactions and pathways resulting in the breakdown of a phenol, any compound containing one or more hydroxyl groups directly attached to an aromatic carbon ring, in the absence of oxygen. Sources: GOC:ai